N-acetylgalactosamine kinase activity [GO:0033858] (molecular function) Also known as: ATP:N-acetyl-D-galactosamine 1-phosphotransferase activity, GALK2, GK2, GalNAc kinase activity, N-acetylgalactosamine (GalNAc)-1-phosphate kinase activity Relationships: is_a GO:0016773; is a type of GO:0019200 Sources: EC:2.7.1.157 Definition: Catalysis of the reaction: ATP + N-acetyl-D-galactosamine = ADP + N-acetyl-alpha-D-galactosamine 1-phosphate.